positive regulation of T-helper 1 type immune response [GO:0002827] (biological process) Relationships: is a type of positive regulation of adaptive immune response based on somatic recombination of immune receptors built from immunoglobulin superfamily domains [GO:0002824]; is a type of GO:0002825; positively regulates T-helper 1 type immune response [GO:0042088] Subtypes: GO:2000556 Sources: GOC:add Definition: Any process that activates or increases the frequency, rate, or extent of a T-helper 1 type immune response. Also known as: up regulation of T-helper 1 type immune response, up-regulation of T-helper 1 type immune response, upregulation of T-helper 1 type immune response, activation of T-helper 1 type immune response, stimulation of T-helper 1 type immune response